{
  "term_id": "UNKNOWN:0001",
  "gene_name": "Putative transporter SVOPL",
  "gene": "UniProtKB:Q8N434",
  "gene_symbol": "SVOPL",
  "term_label": "Unknown molecular function"
}